{
  "term_label": "basement membrane organization",
  "term_id": "GO:0071711",
  "gene_symbol": "PHLDB2",
  "gene_name": "Pleckstrin homology-like domain family B member 2",
  "gene": "UniProtKB:Q86SQ0"
}